peptidyl-glutamic acid carboxylation [GO:0017187] (biological process) Definition: The gamma-carboxylation of peptidyl-glutamic acid; catalyzed by the vitamin K dependent gamma-glutamyl carboxylase. Relationships: is a type of peptidyl-glutamic acid modification [GO:0018200]; is a type of GO:0018214 Note: See also the molecular function term 'gamma-glutamyl carboxylase activity ; GO:0008488'. Sources: RESID:AA0032